{
  "term_label": "plasma membrane",
  "gene": "UniProtKB:O75916",
  "gene_name": "Regulator of G-protein signaling 9",
  "term_id": "GO:0005886",
  "gene_symbol": "RGS9"
}